{
  "term_label": "RNA polymerase II cis-regulatory region sequence-specific DNA binding",
  "gene_name": "Zinc finger and BTB domain-containing protein 37",
  "gene_symbol": "ZBTB37",
  "gene": "UniProtKB:Q5TC79",
  "term_id": "GO:0000978"
}